{
  "gene_name": "Transmembrane protein 39A",
  "gene": "UniProtKB:Q9NV64",
  "term_id": "GO:0005789",
  "gene_symbol": "TMEM39A",
  "term_label": "endoplasmic reticulum membrane"
}